lipoprotein carrier activity [GO:0140598] (molecular function) Definition: Binding to and carrying a lipoprotein between two different cellular locations by moving along with the target lipoprotein. Relationships: is a type of GO:0140597 References: PMID:7628437